{
  "term_label": "Unknown biological process",
  "gene": "UniProtKB:P52943",
  "term_id": "UNKNOWN:0002",
  "gene_name": "Cysteine-rich protein 2",
  "gene_symbol": "CRIP2"
}